{
  "gene": "UniProtKB:Q9P2U8",
  "gene_symbol": "SLC17A6",
  "term_label": "L-glutamate transmembrane transporter activity",
  "gene_name": "Vesicular glutamate transporter 2",
  "term_id": "GO:0005313"
}